{
  "term_id": "GO:0005829",
  "gene": "UniProtKB:Q6P3S1",
  "gene_name": "DENN domain-containing protein 1B",
  "gene_symbol": "DENND1B",
  "term_label": "cytosol"
}